{
  "term_id": "GO:0005634",
  "gene_symbol": "PRKRA",
  "gene_name": "Interferon-inducible double-stranded RNA-dependent protein kinase activator A",
  "gene": "UniProtKB:O75569",
  "term_label": "nucleus"
}